{
  "term_label": "spindle assembly",
  "term_id": "GO:0051225",
  "gene_name": "HAUS augmin-like complex subunit 3",
  "gene": "UniProtKB:Q68CZ6",
  "gene_symbol": "HAUS3"
}